regulation of axon extension involved in regeneration [GO:0048690] (biological process) Relationships: is a type of regulation of axon extension [GO:0030516]; is a type of GO:0048686; regulates axon extension involved in regeneration [GO:0048677] Subtypes: GO:0048691, negative regulation of axon extension involved in regeneration [GO:0048692] Definition: Any process that modulates the frequency, rate or extent of axon extension involved in regeneration. Sources: GOC:dgh, GOC:dph, GOC:jid, GOC:lm